segment polarity determination [GO:0007367] (biological process) Sources: ISBN:0632030488, ISBN:0879694238, http://fly.ebi.ac.uk/allied-data/lk/interactive-fly/aimain/1aahome.htm Relationships: is a type of periodic partitioning [GO:0007365] Definition: Division of the 14 parasegments of the embryo into anterior and posterior compartments; exemplified by the actions of the segment polarity gene products.